{
  "term_label": "muscle contraction",
  "gene_symbol": "MYH2",
  "gene": "UniProtKB:Q9UKX2",
  "gene_name": "Myosin-2",
  "term_id": "GO:0006936"
}